{
  "gene_name": "Helicase SRCAP",
  "term_id": "GO:0006338",
  "gene": "UniProtKB:Q6ZRS2",
  "term_label": "chromatin remodeling",
  "gene_symbol": "SRCAP"
}